sucrose phosphorylase activity [GO:0009018] (molecular function) Relationships: is a type of 1,4-alpha-oligoglucan phosphorylase activity [GO:0004645] Also known as: disaccharide glucosyltransferase activity, sucrose glucosyltransferase activity, sucrose:phosphate alpha-D-glucosyltransferase activity Definition: Catalysis of the reaction: sucrose + phosphate = D-fructose + alpha-D-glucose 1-phosphate. Sources: RHEA:24048